regulation of oligodendrocyte progenitor proliferation [GO:0070445] (BP) Also known as: regulation of oligodendrocyte precursor proliferation Sources: GOC:mah, GOC:sl Relationships: is a type of regulation of neural precursor cell proliferation [GO:2000177]; regulates oligodendrocyte progenitor proliferation [GO:0070444] Subtypes: negative regulation of oligodendrocyte progenitor proliferation [GO:0070446], positive regulation of oligodendrocyte progenitor proliferation [GO:0070447] Definition: Any process that modulates the frequency, rate or extent of oligodendrocyte progenitor proliferation.